posterior neural plate formation [GO:0090018] (biological process) Definition: The formation of posterior end of the flat, thickened layer of ectodermal cells known as the neural plate. Regulation: RO_0002213 by positive regulation of posterior neural plate formation by fibroblast growth factor receptor signaling pathway [GO:0060787] Relationships: is_a anatomical structure formation involved in morphogenesis [GO:0048646]; is part of neural plate formation [GO:0021990] Sources: GOC:dph, GOC:sdb_2009, GOC:tb